{
  "gene": "UniProtKB:P31995",
  "gene_symbol": "FCGR2C",
  "term_label": "cell surface receptor signaling pathway",
  "term_id": "GO:0007166",
  "gene_name": "Low affinity immunoglobulin gamma Fc region receptor II-c"
}